{
  "gene": "UniProtKB:Q9NQ50",
  "term_id": "GO:0005761",
  "term_label": "mitochondrial ribosome",
  "gene_symbol": "MRPL40",
  "gene_name": "Large ribosomal subunit protein mL40"
}